3-hydroxy-2-methylpyridinecarboxylate dioxygenase activity [GO:0047081] (molecular function) Sources: EC:1.14.13.242, MetaCyc:1.14.12.4-RXN Definition: Catalysis of the reaction: O2 + NADPH + H+ + 3-hydroxy-2-methylpyridine-5-carboxylate = NADP+ + 2-(acetamidomethylene)succinate. Also known as: 2-methyl-3-hydroxypyridine 5-carboxylic acid dioxygenase activity, 3-hydroxy-2-methylpyridine-5-carboxylate,NADPH:oxygen oxidoreductase (decyclizing), 3-hydroxy-3-methylpyridinecarboxylate dioxygenase activity, methylhydroxypyridine carboxylate dioxygenase activity, methylhydroxypyridinecarboxylate oxidase activity Relationships: is a type of oxidoreductase activity, acting on paired donors, with incorporation or reduction of molecular oxygen, NAD(P)H as one donor, and incorporation of two atoms of oxygen into one donor [GO:0016708]